{
  "gene_symbol": "AGPAT4",
  "gene": "UniProtKB:Q9NRZ5",
  "term_id": "UNKNOWN:0002",
  "gene_name": "1-acyl-sn-glycerol-3-phosphate acyltransferase delta",
  "term_label": "Unknown biological process"
}